dipeptidyl-peptidase activity [GO:0008239] (molecular function) Sources: GOC:mb, https://www.ebi.ac.uk/merops/about/glossary.shtml#DIPEPTIDYL-PEPTIDASE Relationships: is a type of exopeptidase activity [GO:0008238] Definition: Catalysis of the hydrolysis of N-terminal dipeptides from a polypeptide chain.